G protein-coupled GABA receptor binding [GO:0031795] (molecular function) Definition: Binding to a G protein-coupled (metabotropic) GABA receptor. Sources: GOC:mah, GOC:nln Also known as: G-protein coupled GABA receptor binding, GABAB receptor binding, metabotropic GABA receptor binding, metabotropic GABA receptor ligand Relationships: is a type of G protein-coupled receptor binding [GO:0001664]; is a type of GABA receptor binding [GO:0050811] Subtypes: type 1 metabotropic GABA receptor binding [GO:0031796], type 2 metabotropic GABA receptor binding [GO:0031797]